{
  "gene": "UniProtKB:Q5VW32",
  "term_id": "UNKNOWN:0003",
  "term_label": "Unknown cellular component",
  "gene_symbol": "BROX",
  "gene_name": "BRO1 domain-containing protein BROX"
}